{
  "gene_symbol": "BNIP3",
  "term_label": "mitochondrial outer membrane",
  "gene": "UniProtKB:Q12983",
  "gene_name": "BCL2_adenovirus E1B 19 kDa protein-interacting protein 3",
  "term_id": "GO:0005741"
}